response to dopamine [GO:1903350] (biological process) Relationships: is a type of response to catecholamine [GO:0071869] Subtypes: cellular response to dopamine [GO:1903351] References: PMID:11118945 Sources: GOC:TermGenie, GOC:mr, GO_REF:0000071 Definition: Any process that results in a change in state or activity of a cell or an organism (in terms of movement, secretion, enzyme production, gene expression, etc.) as a result of a dopamine stimulus.